{
  "term_label": "negative regulation of canonical NF-kappaB signal transduction",
  "gene_name": "TNFAIP3-interacting protein 1",
  "gene": "UniProtKB:Q15025",
  "gene_symbol": "TNIP1",
  "term_id": "GO:0043124"
}